regulation of engulfment of apoptotic cell [GO:1901074] (biological process) Also known as: regulation of engulfment of apoptotic cell corpse, regulation of engulfment of cell corpse Relationships: is a type of regulation of phagocytosis, engulfment [GO:0060099]; regulates engulfment of apoptotic cell [GO:0043652] Subtypes: GO:1901075, positive regulation of engulfment of apoptotic cell [GO:1901076] Definition: Any process that modulates the frequency, rate or extent of engulfment of apoptotic cell. References: PMID:19402756 Sources: GO:kmv, GOC:TermGenie